positive regulation of DNA recombination at telomere [GO:0072696] (biological process) Sources: GOC:mah Definition: Any process that activates or increases the frequency, rate or extent of DNA recombination within the telomere. Also known as: positive regulation of telomeric recombination, up regulation of telomeric recombination at telomere, up-regulation of telomeric recombination at telomere, upregulation of telomeric recombination at telomere, activation of telomeric recombination at telomere Relationships: is a type of GO:0045911; is a type of regulation of DNA recombination at telomere [GO:0072695] Subtypes: positive regulation of telomere maintenance via recombination [GO:0032209]